catecholamine secretion [GO:0050432] (biological process) Definition: The regulated release of catecholamines by a cell. The catecholamines are a group of physiologically important biogenic amines that possess a catechol (3,4-dihydroxyphenyl) nucleus and are derivatives of 3,4-dihydroxyphenylethylamine. Sources: GOC:ai, GOC:ef Subtypes: dopamine secretion [GO:0014046], epinephrine secretion [GO:0048242], norepinephrine secretion [GO:0048243], catecholamine secretion, neurotransmission [GO:0160043] Relationships: is a type of secretion by cell [GO:0032940]; is_a catecholamine transport [GO:0051937] Regulation: negatively regulated by negative regulation of catecholamine secretion [GO:0033604]; positively regulated by GO:0033605; regulated by GO:0050433